{
  "term_label": "antigen processing and presentation of exogenous peptide antigen via MHC class II",
  "gene_name": "HLA class II histocompatibility antigen, DR beta 3 chain",
  "term_id": "GO:0019886",
  "gene_symbol": "HLA-DRB3",
  "gene": "UniProtKB:P79483"
}